{
  "term_label": "phosphatidylinositol phosphate binding",
  "gene": "UniProtKB:Q641Q2",
  "term_id": "GO:1901981",
  "gene_name": "WASH complex subunit 2A",
  "gene_symbol": "WASHC2A"
}